Golgi trans cisterna [GO:0000138] (cellular component) Definition: The Golgi cisterna farthest from the endoplasmic reticulum; the final processing compartment through which proteins pass before exiting the Golgi apparatus; the compartment in which N-linked protein glycosylation is completed. Also known as: late Golgi Relationships: is a type of GO:0031985 Sources: ISBN:0815316194